glycosylceramide flippase activity [GO:0140351] (molecular function) References: PMID:30530492 Relationships: is a type of sphingolipid transporter activity [GO:0046624]; is a type of GO:0140327 Also known as: glycoceramide flippase activity, glycosylceramide flippase activity (exoplasmic to cytosolic leaflet), galactocerebroside flippase activity, galactosylceramide flippase activity, glucosylceramide flippase activity Definition: Catalysis of the movement of glycosylceramide from the exoplasmic to the cytosolic leaflet of a membrane, using energy from the hydrolysis of ATP. Glycosylceramides are ceramides containing a functional group derived from a sugar.